{
  "gene_symbol": "ALOXE3",
  "gene": "UniProtKB:Q9BYJ1",
  "term_label": "linoleic acid metabolic process",
  "gene_name": "Hydroperoxide isomerase ALOXE3",
  "term_id": "GO:0043651"
}